{
  "gene_name": "Olfactory receptor 52L1",
  "term_label": "plasma membrane",
  "gene_symbol": "OR52L1",
  "gene": "UniProtKB:Q8NGH7",
  "term_id": "GO:0005886"
}